regulation of L-ascorbic acid biosynthetic process [GO:2000082] (biological process) Also known as: regulation of L-ascorbic acid anabolism, regulation of L-ascorbic acid biosynthesis, regulation of L-ascorbic acid formation, regulation of L-ascorbic acid synthesis, regulation of ascorbate biosynthesis, regulation of ascorbate biosynthetic process, regulation of vitamin C biosynthesis, regulation of vitamin C biosynthetic process Relationships: is a type of regulation of ketone metabolic process [GO:0010565]; is a type of regulation of vitamin metabolic process [GO:0030656]; is a type of regulation of carbohydrate biosynthetic process [GO:0043255]; regulates GO:0019853 Definition: Any process that modulates the frequency, rate or extent of L-ascorbic acid biosynthetic process. Subtypes: GO:2000083 References: PMID:19395407